{
  "term_id": "GO:0060396",
  "gene_name": "Somatotropin",
  "term_label": "growth hormone receptor signaling pathway",
  "gene_symbol": "GH1",
  "gene": "UniProtKB:P01241"
}